{
  "gene_name": "Patched domain-containing protein 1",
  "gene": "UniProtKB:Q96NR3",
  "term_id": "GO:0050890",
  "term_label": "cognition",
  "gene_symbol": "PTCHD1"
}